{
  "gene": "UniProtKB:Q86WC6",
  "term_label": "Unknown biological process",
  "term_id": "UNKNOWN:0002",
  "gene_symbol": "PPP1R27",
  "gene_name": "Protein phosphatase 1 regulatory subunit 27"
}